{
  "term_id": "GO:0055056",
  "gene_name": "Solute carrier family 2, facilitated glucose transporter member 7",
  "term_label": "D-glucose transmembrane transporter activity",
  "gene": "UniProtKB:Q6PXP3",
  "gene_symbol": "SLC2A7"
}